{
  "gene_name": "Chromodomain-helicase-DNA-binding protein 3",
  "gene_symbol": "CHD3",
  "term_label": "ATP hydrolysis activity",
  "gene": "UniProtKB:Q12873",
  "term_id": "GO:0016887"
}